{
  "gene_name": "Putative sodium-coupled neutral amino acid transporter 11",
  "gene": "UniProtKB:Q08AI6",
  "gene_symbol": "SLC38A11",
  "term_id": "GO:0016020",
  "term_label": "membrane"
}